glucarate biosynthetic process [GO:0019393] (biological process) Relationships: is a type of aldaric acid biosynthetic process [GO:0019578] Definition: The chemical reactions and pathways resulting in the formation of glucarate, the anion of glucaric acid. Also known as: glucarate anabolism, glucarate biosynthesis, glucarate formation, glucarate synthesis Subtypes: D-glucarate biosynthetic process [GO:0042837] Sources: ISBN:0198506732